abietadiene synthase activity [GO:0050554] (molecular function) Also known as: (+)-copalyl-diphosphate diphosphate-lyase (cyclizing, (-)-abietadiene-forming), abietadiene cyclase activity, copalyl-diphosphate diphosphate-lyase (cyclizing) Relationships: is a type of carbon-oxygen lyase activity, acting on phosphates [GO:0016838] Sources: EC:4.2.3.18, RHEA:13873 Definition: Catalysis of the reaction: (+)-copalyl diphosphate = (-)-abietadiene + diphosphate.